{
  "gene": "UniProtKB:Q8N402",
  "gene_symbol": "Q8N402",
  "term_label": "Unknown molecular function",
  "term_id": "UNKNOWN:0001",
  "gene_name": "Putative uncharacterized protein LOC388882"
}